{
  "gene_symbol": "TM9SF3",
  "term_id": "GO:0072657",
  "term_label": "protein localization to membrane",
  "gene": "UniProtKB:Q9HD45",
  "gene_name": "Transmembrane 9 superfamily member 3"
}